fatty acid elongation, monounsaturated fatty acid [GO:0034625] (biological process) Definition: Elongation of a fatty acid chain into which one C-C double bond has been introduced. Relationships: is a type of fatty acid elongation, unsaturated fatty acid [GO:0019368] Sources: GOC:mah